regulation of mitotic nuclear division [GO:0007088] (biological process) Subtypes: GO:0045839, positive regulation of mitotic nuclear division [GO:0045840], regulation of mitotic cell cycle spindle assembly checkpoint [GO:0090266] Sources: GOC:go_curators Definition: Any process that modulates the frequency, rate or extent of mitosis. Also known as: regulation of mitosis Relationships: is a type of regulation of mitotic cell cycle [GO:0007346]; is a type of GO:0010564; is a type of regulation of nuclear division [GO:0051783]; regulates mitotic nuclear division [GO:0140014]